{
  "term_id": "GO:0005886",
  "gene_symbol": "KCNT1",
  "gene": "UniProtKB:Q5JUK3",
  "term_label": "plasma membrane",
  "gene_name": "Potassium channel subfamily T member 1"
}